{
  "gene_name": "Regulation of nuclear pre-mRNA domain-containing protein 1B",
  "gene_symbol": "RPRD1B",
  "term_label": "RNA polymerase II complex binding",
  "gene": "UniProtKB:Q9NQG5",
  "term_id": "GO:0000993"
}